regulation of cardiac muscle contraction [GO:0055117] (biological process) Definition: Any process that modulates the frequency, rate or extent of cardiac muscle contraction. Sources: GOC:ecd Relationships: is a type of regulation of striated muscle contraction [GO:0006942]; is a type of regulation of heart contraction [GO:0008016]; regulates cardiac muscle contraction [GO:0060048] Subtypes: regulation of cardiac muscle contraction by calcium ion signaling [GO:0010882], negative regulation of cardiac muscle contraction [GO:0055118], GO:0060452, regulation of cardiac muscle cell contraction [GO:0086004]